neuroblast division in subventricular zone [GO:0021849] (biological process) Definition: The division of neuroblasts in the subventricular zone of the forebrain. The interneuron precursors that these cells give rise to include adult olfactory bulb interneurons and migrate tangentially. References: PMID:12626695 Sources: GOC:cls, GOC:dgh, GOC:dph, GOC:jid, GO_REF:0000021 Relationships: is a type of neuroblast division [GO:0055057]; is part of cell proliferation in forebrain [GO:0021846]